{
  "term_id": "GO:0032580",
  "term_label": "Golgi cisterna membrane",
  "gene_symbol": "GOLGA8K",
  "gene": "UniProtKB:D6RF30",
  "gene_name": "Golgin subfamily A member 8K"
}